{
  "term_id": "GO:1902600",
  "term_label": "proton transmembrane transport",
  "gene": "UniProtKB:P54707",
  "gene_symbol": "ATP12A",
  "gene_name": "Potassium-transporting ATPase alpha chain 2"
}